{
  "gene_symbol": "LTF",
  "gene_name": "Lactotransferrin",
  "term_label": "early endosome",
  "term_id": "GO:0005769",
  "gene": "UniProtKB:P02788"
}